{
  "gene": "UniProtKB:Q96G79",
  "term_label": "Golgi membrane",
  "term_id": "GO:0000139",
  "gene_name": "Probable UDP-sugar transporter protein SLC35A4",
  "gene_symbol": "SLC35A4"
}